regulation of cytokinesis, site selection [GO:2000073] (biological process) Sources: GOC:mtg_cell_cycle, GOC:obol Subtypes: regulation of mitotic cytokinesis, division site positioning [GO:1902472], negative regulation of cytokinesis, site selection [GO:2000075], positive regulation of cytokinesis, site selection [GO:2000076] Relationships: is a type of GO:0032954; regulates cytokinesis, division site positioning [GO:0007105] Also known as: regulation of site selection involved in cell cycle cytokinesis Definition: Any process that modulates the frequency, rate or extent of site selection that occurs as part of cytokinesis.